{
  "term_label": "prostaglandin-I synthase activity",
  "gene_symbol": "PTGIS",
  "gene": "UniProtKB:Q16647",
  "term_id": "GO:0008116",
  "gene_name": "Prostacyclin synthase"
}